notum morphogenesis [GO:0048802] (BP) Sources: GOC:jid Definition: The process in which the anatomical structures of the dorsal part of the body are generated and organized. Relationships: is a type of GO:0009886; is part of wing disc morphogenesis [GO:0007472]; is part of notum development [GO:0007477]